{
  "gene": "UniProtKB:Q5VVY1",
  "gene_symbol": "NTMT2",
  "term_id": "GO:0071885",
  "gene_name": "N-terminal Xaa-Pro-Lys N-methyltransferase 2",
  "term_label": "N-terminal protein N-methyltransferase activity"
}